positive regulation of auxin metabolic process [GO:0090355] (biological process) Relationships: is a type of positive regulation of hormone metabolic process [GO:0032352]; is a type of regulation of auxin metabolic process [GO:0090354]; positively regulates auxin metabolic process [GO:0009850] Definition: Any process that increases the frequency, rate or extent of the chemical reactions and pathways involving auxins, plant hormones that regulate aspects of plant growth. Sources: GOC:tb Subtypes: GO:0010601 Also known as: positive regulation of auxin metabolism